prostaglandin H2 endoperoxidase reductase activity [GO:0036130] (molecular function) Relationships: is a type of GO:0016616; is part of prostaglandin metabolic process [GO:0006693] Definition: Catalysis of the reaction: prostaglandin F2alpha + NADP+ = prostaglandin H2 + NADPH + H+. References: PMID:10622721, PMID:14979715, PMID:16475787 Sources: RHEA:45312 Also known as: PGH2 9,11-endoperoxidase, PGH2 9-,11-endoperoxide reductase